{
  "term_label": "regulation of gene expression",
  "gene": "UniProtKB:P16989",
  "term_id": "GO:0010468",
  "gene_name": "Y-box-binding protein 3",
  "gene_symbol": "YBX3"
}